{
  "term_label": "Unknown molecular function",
  "gene_name": "Zinc finger protein 230",
  "term_id": "UNKNOWN:0001",
  "gene": "UniProtKB:Q9UIE0",
  "gene_symbol": "ZNF230"
}